octanoic acid binding [GO:1904767] (molecular function) References: PMID:19828452 Sources: GOC:TermGenie, GOC:kmv, GO_REF:0000067 Relationships: is a type of GO:0005504 Definition: Binding to octanoic acid. Also known as: caprylic acid binding